protein transport within lipid bilayer [GO:0032594] (biological process) Relationships: is a type of intracellular protein transport [GO:0006886]; is a type of GO:0061024; occurs in GO:0016020 Subtypes: B cell receptor transport within lipid bilayer [GO:0032595], protein transport into membrane raft [GO:0032596], GO:0032599, chemokine receptor transport within lipid bilayer [GO:0033606], protein transport within plasma membrane [GO:0099632], protein transport from ciliary membrane to plasma membrane [GO:1903445] Definition: The directed movement of a protein from one location to another within a lipid bilayer. Sources: GOC:mah Also known as: protein translocation within membrane, receptor translocation within membrane, receptor transport within lipid bilayer